serotonin secretion by mast cell [GO:0002552] (biological process) Sources: GOC:add, ISBN:0781735149 Definition: The regulated release of serotonin by a mast cell or group of mast cells. Also known as: serotonin release by mast cell Relationships: is a type of serotonin secretion involved in inflammatory response [GO:0002442]; is a type of establishment of localization in cell [GO:0051649]; is a type of exocytic process [GO:0140029]; is part of GO:0043303